long nephron development [GO:0072029] (biological process) Sources: GOC:mtg_kidney_jan10 Subtypes: metanephric long nephron development [GO:0072238] Also known as: juxtamedullary nephron development Definition: The process whose specific outcome is the progression of a long nephron over time, from its formation to the mature structure. Long nephrons are associated with juxtamedullary glomeruli and extend into the inner medulla. Relationships: is a type of nephron development [GO:0072006]